{
  "gene_name": "Cadherin-8",
  "gene_symbol": "CDH8",
  "gene": "UniProtKB:P55286",
  "term_label": "calcium-dependent cell-cell adhesion",
  "term_id": "GO:0016339"
}